{
  "term_id": "GO:0006303",
  "gene_symbol": "DCLRE1A",
  "gene": "UniProtKB:Q6PJP8",
  "term_label": "double-strand break repair via nonhomologous end joining",
  "gene_name": "DNA cross-link repair 1A protein"
}